{
  "term_id": "GO:0005504",
  "gene_symbol": "ACOX2",
  "term_label": "fatty acid binding",
  "gene": "UniProtKB:Q99424",
  "gene_name": "Peroxisomal acyl-coenzyme A oxidase 2"
}